{
  "gene_name": "Olfactory receptor 5B12",
  "term_label": "G protein-coupled receptor signaling pathway",
  "gene_symbol": "OR5B12",
  "gene": "UniProtKB:Q96R08",
  "term_id": "GO:0007186"
}